nucleoside triphosphate metabolic process [GO:0009141] (biological process) Definition: The chemical reactions and pathways involving a nucleoside triphosphate, a compound consisting of a nucleobase linked to a deoxyribose or ribose sugar esterified with triphosphate on the sugar. Sources: GOC:go_curators, ISBN:0198506732 Also known as: nucleoside triphosphate metabolism Relationships: is a type of GO:0006753 Subtypes: nucleoside triphosphate biosynthetic process [GO:0009142], nucleoside triphosphate catabolic process [GO:0009143], purine nucleoside triphosphate metabolic process [GO:0009144], pyrimidine nucleoside triphosphate metabolic process [GO:0009147], deoxyribonucleoside triphosphate metabolic process [GO:0009200]